{
  "gene_name": "Putative uncharacterized protein encoded by LINC00269",
  "term_label": "Unknown cellular component",
  "gene": "UniProtKB:Q8N2A0",
  "gene_symbol": "LINC00269",
  "term_id": "UNKNOWN:0003"
}